{
  "gene_symbol": "MAP1S",
  "gene_name": "Microtubule-associated protein 1S",
  "term_label": "microtubule associated complex",
  "gene": "UniProtKB:Q66K74",
  "term_id": "GO:0005875"
}